host-mediated suppression of viral transcription [GO:0043922] (biological process) Also known as: negative regulation by host of viral transcription, negative regulation of viral transcription by host Sources: GOC:jl Definition: A process in which a host organism interferes with, inhibits or disrupts viral transcription. Relationships: is a type of host-mediated perturbation of viral transcription [GO:0043921]; is a type of host-mediated suppression of viral proces [GO:0044793]